{
  "gene_name": "Transcription factor AP-2-delta",
  "term_label": "RNA polymerase II transcription regulatory region sequence-specific DNA binding",
  "term_id": "GO:0000977",
  "gene_symbol": "TFAP2D",
  "gene": "UniProtKB:Q7Z6R9"
}